{
  "gene_symbol": "S100A1",
  "gene_name": "Protein S100-A1",
  "gene": "UniProtKB:P23297",
  "term_label": "calcium ion binding",
  "term_id": "GO:0005509"
}